{
  "gene": "UniProtKB:Q13347",
  "term_id": "GO:0002183",
  "gene_symbol": "EIF3I",
  "gene_name": "Eukaryotic translation initiation factor 3 subunit I",
  "term_label": "cytoplasmic translational initiation"
}